UDPsulfoquinovose synthase activity [GO:0046507] (molecular function) Definition: Catalysis of the reaction: sulfite + UDP-D-glucose = H2O + UDP-6-sulfoquinovose. Sources: EC:3.13.1.1, RHEA:13197 Relationships: is a type of hydrolase activity, acting on carbon-sulfur bonds [GO:0046508] Also known as: UDPsulphoquinovose synthase activity, sulfite:UDP-glucose sulfotransferase activity, UDP-6-sulfo-6-deoxyglucose sulfohydrolase activity, UDP-sulfoquinovose synthase activity